{
  "gene_symbol": "NOMO3",
  "term_label": "Unknown biological process",
  "gene": "UniProtKB:P69849",
  "term_id": "UNKNOWN:0002",
  "gene_name": "BOS complex subunit NOMO3"
}